{
  "term_id": "GO:0006357",
  "gene": "UniProtKB:Q6ZS27",
  "term_label": "regulation of transcription by RNA polymerase II",
  "gene_symbol": "ZNF662",
  "gene_name": "Zinc finger protein 662"
}